{
  "term_id": "GO:0005737",
  "gene_name": "Growth arrest and DNA damage-inducible protein GADD45 beta",
  "gene_symbol": "GADD45B",
  "gene": "UniProtKB:O75293",
  "term_label": "cytoplasm"
}